{
  "term_id": "GO:0006338",
  "term_label": "chromatin remodeling",
  "gene": "UniProtKB:Q58F21",
  "gene_symbol": "BRDT",
  "gene_name": "Bromodomain testis-specific protein"
}